{
  "gene_symbol": "TNN",
  "term_label": "extracellular space",
  "gene": "UniProtKB:Q9UQP3",
  "gene_name": "Tenascin-N",
  "term_id": "GO:0005615"
}